ribonucleoprotein complex binding [GO:0043021] (molecular function) Subtypes: signal recognition particle binding [GO:0005047], snoRNP binding [GO:0030519], ribosome binding [GO:0043022], snRNP binding [GO:0070990], RISC complex binding [GO:1905172], preribosome binding [GO:1990275] Relationships: is a type of protein-containing complex binding [GO:0044877] Sources: GOC:bf, GOC:go_curators, GOC:vk Definition: Binding to a complex of RNA and protein. Also known as: RNP binding, protein-RNA complex binding, ribonucleoprotein binding